transferrin receptor activity [GO:0004998] (molecular function) References: PMID:2678449, PMID:3011819 Sources: GOC:bf Definition: Combining selectively with transferrin, and delivering transferrin into the cell via endocytosis. Transferrin is a major iron carrier protein in vertebrates. Relationships: is a type of cargo receptor activity [GO:0038024]